{
  "term_label": "calcium channel inhibitor activity",
  "gene_name": "Proton-coupled zinc antiporter SLC30A1",
  "term_id": "GO:0019855",
  "gene_symbol": "SLC30A1",
  "gene": "UniProtKB:Q9Y6M5"
}